{
  "gene": "UniProtKB:O75676",
  "term_id": "GO:0038202",
  "gene_symbol": "RPS6KA4",
  "term_label": "TORC1 signaling",
  "gene_name": "Ribosomal protein S6 kinase alpha-4"
}